{
  "gene_symbol": "THRAP3",
  "term_id": "GO:0016592",
  "gene": "UniProtKB:Q9Y2W1",
  "gene_name": "Thyroid hormone receptor-associated protein 3",
  "term_label": "mediator complex"
}